vitelline membrane formation involved in chorion-containing eggshell formation [GO:0007305] (biological process) Definition: Construction of the vitelline membrane portion of a chorion-containing eggshell. An example of this is found in Drosophila melanogaster. Sources: GOC:mah, GOC:mtg_sensu Also known as: vitelline membrane formation in chorion-containing eggshell Relationships: is a type of vitelline membrane formation [GO:0030704]; is part of GO:0007304